{
  "gene_symbol": "PAX1",
  "gene": "UniProtKB:P15863",
  "term_label": "regulation of transcription by RNA polymerase II",
  "gene_name": "Paired box protein Pax-1",
  "term_id": "GO:0006357"
}